acceptance of pollen [GO:0060321] (biological process) Definition: The recognition and acceptance of pollen by cells in the stigma, mediated by the sharing and interaction of the single locus incompatibility haplotypes. Relationships: is a type of GO:0048544; is part of pollen-pistil interaction [GO:0009875] Also known as: acceptance of self pollen, acceptance of non-self pollen, self-compatibility Sources: GOC:dph, GOC:tb